(R)-carnitine transport [GO:1900749] (biological process) Also known as: (3R)-3-hydroxy-4-(trimethylammonio)butanoate transport, L-Carnitine transport, (-)-Carnitine transport, (-)-L-Carnitine transport, C7H15NO3 transport, Carnicor transport, Carnitene transport, Carnitine transport, Carnitor transport, Levocarnitine transport, Vitamin BT transport References: PMID:16365044, PMID:20357772, PMID:20829798 Sources: GOC:TermGenie Subtypes: (R)-carnitine transmembrane transport [GO:1902270] Definition: The directed movement of a (R)-carnitine into, out of or within a cell, or between cells, by means of some agent such as a transporter or pore. Relationships: is a type of GO:0015879